{
  "term_label": "GTPase activator activity",
  "term_id": "GO:0005096",
  "gene_name": "Regulator of G-protein signaling 12",
  "gene": "UniProtKB:O14924",
  "gene_symbol": "RGS12"
}